formate transmembrane transporter activity [GO:0015499] (molecular function) Also known as: formate uptake permease activity, formate uptake transmembrane transporter activity Sources: GOC:ai Subtypes: formate efflux transmembrane transporter activity [GO:0015660] Definition: Enables the transfer of formate from one side of a membrane to the other. Formate is also known as methanoate, the anion HCOO- derived from methanoic (formic) acid. Relationships: is a type of monocarboxylic acid transmembrane transporter activity [GO:0008028]; is part of formate transport [GO:0015724]